{
  "gene_name": "Receptor tyrosine-protein kinase erbB-3",
  "term_id": "GO:0043066",
  "gene_symbol": "ERBB3",
  "gene": "UniProtKB:P21860",
  "term_label": "negative regulation of apoptotic process"
}